{
  "gene": "UniProtKB:O94856",
  "term_label": "plasma membrane",
  "gene_name": "Neurofascin",
  "gene_symbol": "NFASC",
  "term_id": "GO:0005886"
}